{
  "gene": "UniProtKB:O95208",
  "gene_name": "Epsin-2",
  "term_id": "GO:0030125",
  "gene_symbol": "EPN2",
  "term_label": "clathrin vesicle coat"
}